{
  "term_id": "GO:0004674",
  "gene_symbol": "PRKD1",
  "gene": "UniProtKB:Q15139",
  "gene_name": "Serine_threonine-protein kinase D1",
  "term_label": "protein serine/threonine kinase activity"
}